arbutin transport [GO:0042949] (BP) Definition: The directed movement of arbutin, a glycoside found in the bearberry and related plants which has been used to treat urinary-tract diseases, into, out of or within a cell, or between cells, by means of some agent such as a transporter or pore. References: PMID:19965875 Sources: GOC:jl Relationships: is a type of GO:0015759